{
  "gene": "UniProtKB:A6NNB3",
  "gene_name": "Interferon-induced transmembrane protein 5",
  "term_label": "Unknown molecular function",
  "term_id": "UNKNOWN:0001",
  "gene_symbol": "IFITM5"
}